{
  "gene": "UniProtKB:H3BV60",
  "term_label": "regulation of transforming growth factor beta receptor signaling pathway",
  "gene_symbol": "TGFBR3L",
  "gene_name": "Transforming growth factor-beta receptor type 3-like protein",
  "term_id": "GO:0017015"
}